BMP binding [GO:0036122] (molecular function) Relationships: is a type of GO:0019955 Also known as: bone morphogenetic protein binding References: PMID:9660951 Sources: GOC:BHF Definition: Binding to a member of the bone morphogenetic protein (BMP) family.